{
  "term_label": "Unknown biological process",
  "gene": "UniProtKB:O95857",
  "gene_symbol": "TSPAN13",
  "term_id": "UNKNOWN:0002",
  "gene_name": "Tetraspanin-13"
}